organophosphate catabolic process [GO:0046434] (biological process) Also known as: organophosphate breakdown, organophosphate catabolism, organophosphate degradation Subtypes: GO:0009395, parathion catabolic process [GO:0019339], GO:0019664, glyceraldehyde-3-phosphate catabolic process [GO:0019683], molybdopterin cofactor catabolic process [GO:0032325], GO:0032361, galactose catabolic process via UDP-galactose, Leloir pathway [GO:0033499], GO:0042358, phosphagen catabolic process [GO:0042397], glycerol-3-phosphate catabolic process [GO:0046168], deoxyribose phosphate catabolic process [GO:0046386], inositol phosphate catabolic process [GO:0071545], D-ribose 5-phosphate catabolic process [GO:1901279], 5,6,7,8-tetrahydromethanopterin catabolic process [GO:1901284], GO:1901292, GO:1901854, D-tagatose 6-phosphate catabolic process [GO:2001059] Definition: The chemical reactions and pathways resulting in the breakdown of organophosphates, any phosphate-containing organic compound. Sources: GOC:ai Relationships: is a type of catabolic process [GO:0009056]; is a type of organophosphate metabolic process [GO:0019637]